negative regulation of protein localization to cilium [GO:1903565] (biological process) Also known as: down regulation of protein localization to cilium, down-regulation of protein localization to cilium, downregulation of protein localization to cilium, inhibition of protein localization to cilium References: PMID:22072986 Sources: GOC:TermGenie, GOC:cilia, GOC:krc, GO_REF:0000058 Subtypes: GO:1903568 Relationships: is a type of regulation of protein localization to cilium [GO:1903564]; is a type of GO:1903828; negatively regulates protein localization to cilium [GO:0061512] Definition: Any process that stops, prevents or reduces the frequency, rate or extent of protein localization to cilium.